AAA codon-amino acid adaptor activity [GO:0033443] (molecular function) Definition: A triplet codon-amino acid adaptor activity that recognizes an AAA codon. Sources: GOC:mah Also known as: lysine tRNA Note: Note that in the standard genetic code, AAA codes for lysine. Relationships: is a type of triplet codon-amino acid adaptor activity [GO:0030533]